plastid to vacuole vesicle-mediated transport [GO:1904962] (biological process) Definition: The vesicle-mediated and directed movement of substances from plastid to vacuole. References: PMID:25281689 Sources: GOC:TermGenie, GO_REF:0000076 Also known as: plastid to vacuolar carboxypeptidase Y vesicle-mediated transport Relationships: is a type of vacuolar transport [GO:0007034]; is a type of vesicle-mediated transport [GO:0016192]; is a type of cytosolic transport [GO:0016482]